glycolipid transfer activity [GO:0017089] (molecular function) Also known as: glycolipid transporter activity, glycolipid carrier activity, intermembrane glycolipid transfer activity, intermembrane glycolipid transporter activity References: PMID:30337668 Subtypes: cerebroside transfer activity [GO:0140340] Definition: Removes a glycolipid from a membrane or a monolayer lipid particle, transports it through the aqueous phase while protected in a hydrophobic pocket, and brings it to an acceptor membrane or lipid particle. A glycolipid is a compound usually containing 1-4 linked monosaccharide residues joined by a glycosyl linkage to a lipid. Relationships: is a type of GO:0120013; is part of glycolipid transport [GO:0046836]; has part GO:0051861